{
  "gene_name": "Kinesin heavy chain isoform 5A",
  "term_id": "GO:0008574",
  "term_label": "plus-end-directed microtubule motor activity",
  "gene": "UniProtKB:Q12840",
  "gene_symbol": "KIF5A"
}